{
  "gene_name": "Ribonucleoprotein PTB-binding 2",
  "gene": "UniProtKB:Q9HCJ3",
  "term_id": "UNKNOWN:0003",
  "term_label": "Unknown cellular component",
  "gene_symbol": "RAVER2"
}